excretion [GO:0007588] (biological process) Definition: The elimination by an organism of the waste products that arise as a result of metabolic activity. These products include water, carbon dioxide (CO2), and nitrogenous compounds. Sources: ISBN:0192801023 Relationships: is a type of GO:0003008 Subtypes: defecation [GO:0030421], micturition [GO:0060073], renal tubular secretion [GO:0097254], ammonium excretion [GO:0140734] Regulation: regulated by regulation of excretion [GO:0044062]